{
  "gene_symbol": "CHGA",
  "gene_name": "Chromogranin-A",
  "term_id": "UNKNOWN:0001",
  "term_label": "Unknown molecular function",
  "gene": "UniProtKB:P10645"
}